{
  "term_label": "Unknown cellular component",
  "gene_name": "Small proline-rich protein 2B",
  "gene_symbol": "SPRR2B",
  "gene": "UniProtKB:P35325",
  "term_id": "UNKNOWN:0003"
}